{
  "gene": "UniProtKB:Q96CG8",
  "gene_symbol": "CTHRC1",
  "gene_name": "Collagen triple helix repeat-containing protein 1",
  "term_label": "neuron projection",
  "term_id": "GO:0043005"
}